{
  "gene": "UniProtKB:Q8NFU3",
  "gene_symbol": "TSTD1",
  "gene_name": "Thiosulfate:glutathione sulfurtransferase",
  "term_id": "GO:0005737",
  "term_label": "cytoplasm"
}